keratan sulfate proteoglycan biosynthetic process [GO:0018146] (biological process) Also known as: keratan sulfate anabolism, keratan sulfate biosynthesis, keratan sulfate formation, keratan sulfate synthesis, keratan sulphate biosynthesis, keratan sulphate biosynthetic process Definition: The chemical reactions and pathways resulting in the formation of keratan sulfate proteoglycans, which consist of a core protein linked to a keratan sulfate glycosaminoglycan. The keratan sulfate chain is composed of the repeating disaccharide unit beta-(1,4)-N-acetyl-D-glucosamine-beta-(1,3)-galactose, both of which can be sulfated. Keratan sulfate chains can be covalently linked either to an asparagine residue (N-linked) of the core protein via a high mannose oligasacccharide linker or to serine/threonine residues (O-linked) of the core protein via a core 2 type-linker. Subtypes: keratan sulfate-I proteoglycan biosynthetic process [GO:0140263], keratan sulfate-II proteoglycan biosynthetic process [GO:0140264], GO:0140265 Relationships: is a type of GO:0030166; is a type of keratan sulfate proteoglycan metabolic process [GO:0042339] References: PMID:29340594